{
  "term_id": "UNKNOWN:0002",
  "gene": "UniProtKB:P49326",
  "term_label": "Unknown biological process",
  "gene_name": "Flavin-containing monooxygenase 5",
  "gene_symbol": "FMO5"
}